{
  "gene_name": "Sodium_potassium-transporting ATPase subunit alpha-4",
  "gene_symbol": "ATP1A4",
  "gene": "UniProtKB:Q13733",
  "term_label": "potassium ion import across plasma membrane",
  "term_id": "GO:1990573"
}